{
  "gene": "UniProtKB:P62736",
  "gene_symbol": "ACTA2",
  "term_label": "Unknown biological process",
  "term_id": "UNKNOWN:0002",
  "gene_name": "Actin, aortic smooth muscle"
}